{
  "gene_name": "Voltage-dependent L-type calcium channel subunit beta-3",
  "gene_symbol": "CACNB3",
  "term_label": "voltage-gated calcium channel complex",
  "term_id": "GO:0005891",
  "gene": "UniProtKB:P54284"
}